{
  "gene_symbol": "IDH3B",
  "term_label": "mitochondrion",
  "term_id": "GO:0005739",
  "gene": "UniProtKB:O43837",
  "gene_name": "Isocitrate dehydrogenase [NAD] subunit beta, mitochondrial"
}